{
  "gene_name": "Spindlin-1",
  "gene": "UniProtKB:Q9Y657",
  "term_id": "GO:0006355",
  "gene_symbol": "SPIN1",
  "term_label": "regulation of DNA-templated transcription"
}